{
  "term_label": "nucleus",
  "gene": "UniProtKB:A0A087WUV0",
  "term_id": "GO:0005634",
  "gene_symbol": "ZNF892",
  "gene_name": "Zinc finger protein 892"
}